{
  "gene_name": "Cytosolic iron-sulfur assembly component 3",
  "gene": "UniProtKB:Q9H6Q4",
  "term_label": "Unknown molecular function",
  "gene_symbol": "CIAO3",
  "term_id": "UNKNOWN:0001"
}